{
  "term_id": "UNKNOWN:0001",
  "term_label": "Unknown molecular function",
  "gene": "UniProtKB:Q6ZSS7",
  "gene_name": "Major facilitator superfamily domain-containing protein 6",
  "gene_symbol": "MFSD6"
}